{
  "term_label": "intracellular sterol transport",
  "gene": "UniProtKB:Q96CP6",
  "gene_name": "Protein Aster-A",
  "gene_symbol": "GRAMD1A",
  "term_id": "GO:0032366"
}